{
  "gene": "UniProtKB:A0A0C4DH90",
  "term_label": "Unknown molecular function",
  "gene_name": "Immunoglobulin kappa variable 3_OR2-268 (non-functional) (Fragment)",
  "term_id": "UNKNOWN:0001",
  "gene_symbol": "IGKV3OR2-268"
}